{
  "gene_name": "Putative prolyl-tRNA synthetase associated domain-containing protein 1",
  "term_label": "Unknown molecular function",
  "gene": "UniProtKB:A6NEY8",
  "gene_symbol": "PRORSD1P",
  "term_id": "UNKNOWN:0001"
}